2-aminobenzenesulfonate 2,3-dioxygenase activity [GO:0018627] (molecular function) Also known as: 2-aminobenzenesulfonate dioxygenase activity, 2-aminobenzenesulphonate 2,3-dioxygenase activity, 2-aminobenzenesulphonate dioxygenase activity, 2-aminobenzenesulfonate,NADH:oxygen oxidoreductase (2,3-hydroxylating, ammonia-forming), 2-aminosulfobenzene 2,3-dioxygenase activity Relationships: is a type of oxidoreductase activity, acting on paired donors, with incorporation or reduction of molecular oxygen, NAD(P)H as one donor, and incorporation of two atoms of oxygen into one donor [GO:0016708] Sources: EC:1.14.12.14, RHEA:23468 Definition: Catalysis of the reaction: 2-aminobenzenesulfonate + 2 H+ + NADH + O2 = 2,3-dihydroxybenzenesulfonate + NAD+ + NH4. 2,3-dihydroxybenzenesulfonate is also known as 3-sulfocatechol.